{
  "term_id": "UNKNOWN:0003",
  "term_label": "Unknown cellular component",
  "gene_symbol": "EGFL6",
  "gene": "UniProtKB:Q8IUX8",
  "gene_name": "Epidermal growth factor-like protein 6"
}